{
  "gene_name": "E3 ubiquitin-protein ligase SMURF2",
  "term_label": "ubiquitin protein ligase activity",
  "gene_symbol": "SMURF2",
  "term_id": "GO:0061630",
  "gene": "UniProtKB:Q9HAU4"
}